{
  "term_label": "high-affinity IgE receptor activity",
  "gene_symbol": "FCER1A",
  "gene": "UniProtKB:P12319",
  "gene_name": "High affinity immunoglobulin epsilon receptor subunit alpha",
  "term_id": "GO:0019768"
}